{
  "gene_name": "Acetylgalactosaminyl-O-glycosyl-glycoprotein beta-1,3-N-acetylglucosaminyltransferase",
  "gene_symbol": "B3GNT6",
  "gene": "UniProtKB:Q6ZMB0",
  "term_label": "UDP-glycosyltransferase activity",
  "term_id": "GO:0008194"
}